{
  "gene_symbol": "RARG",
  "gene_name": "Retinoic acid receptor gamma",
  "gene": "UniProtKB:P13631",
  "term_label": "RNA polymerase II transcription regulator complex",
  "term_id": "GO:0090575"
}